{
  "term_id": "UNKNOWN:0002",
  "term_label": "Unknown biological process",
  "gene": "UniProtKB:Q8IVU9",
  "gene_symbol": "CABCOCO1",
  "gene_name": "Ciliary-associated calcium-binding coiled-coil protein 1"
}